{
  "gene_name": "Protein ERGIC-53",
  "gene": "UniProtKB:P49257",
  "term_label": "D-mannose binding",
  "gene_symbol": "LMAN1",
  "term_id": "GO:0005537"
}